{
  "gene": "UniProtKB:P01574",
  "term_id": "GO:0002312",
  "gene_name": "Interferon beta",
  "term_label": "B cell activation involved in immune response",
  "gene_symbol": "IFNB1"
}